negative regulation of homoserine biosynthetic process [GO:1901711] (biological process) Sources: GOC:TermGenie Relationships: is a type of negative regulation of small molecule metabolic process [GO:0062014]; is a type of GO:1901710; is a type of negative regulation of amino acid biosynthetic process [GO:2000283]; negatively regulates homoserine biosynthetic process [GO:0009090] Definition: Any process that stops, prevents or reduces the frequency, rate or extent of homoserine biosynthetic process. Also known as: down regulation of homoserine anabolism, down regulation of homoserine biosynthesis, down regulation of homoserine biosynthetic process, down regulation of homoserine formation, down regulation of homoserine synthesis, down-regulation of homoserine anabolism, down-regulation of homoserine biosynthesis, down-regulation of homoserine biosynthetic process, down-regulation of homoserine formation, down-regulation of homoserine synthesis, downregulation of homoserine anabolism, downregulation of homoserine biosynthesis, downregulation of homoserine biosynthetic process, downregulation of homoserine formation, downregulation of homoserine synthesis, inhibition of homoserine anabolism, inhibition of homoserine biosynthesis, inhibition of homoserine formation, inhibition of homoserine synthesis, negative regulation of homoserine anabolism, negative regulation of homoserine biosynthesis, negative regulation of homoserine formation, negative regulation of homoserine synthesis, inhibition of homoserine biosynthetic process